{
  "gene": "UniProtKB:A0A2Z4LIS9",
  "gene_symbol": "FOXO3B",
  "term_id": "GO:0000981",
  "term_label": "DNA-binding transcription factor activity, RNA polymerase II-specific",
  "gene_name": "Forkhead box protein O3B"
}